{
  "gene_name": "Zinc finger protein 566",
  "term_label": "regulation of transcription by RNA polymerase II",
  "term_id": "GO:0006357",
  "gene_symbol": "ZNF566",
  "gene": "UniProtKB:Q969W8"
}